{
  "gene_symbol": "OR8A1",
  "term_label": "Unknown cellular component",
  "term_id": "UNKNOWN:0003",
  "gene": "UniProtKB:Q8NGG7",
  "gene_name": "Olfactory receptor 8A1"
}